{
  "term_id": "GO:0005886",
  "term_label": "plasma membrane",
  "gene_symbol": "HSP90AB1",
  "gene": "UniProtKB:P08238",
  "gene_name": "Heat shock protein HSP 90-beta"
}